negative regulation of intermediate filament depolymerization [GO:0030843] (biological process) Sources: GOC:mah Also known as: negative regulation of intermediate filament polymerization and/or depolymerization, down regulation of intermediate filament depolymerization, down-regulation of intermediate filament depolymerization, downregulation of intermediate filament depolymerization, inhibition of intermediate filament depolymerization Relationships: is a type of regulation of intermediate filament depolymerization [GO:0030842]; is a type of negative regulation of cytoskeleton organization [GO:0051494]; is a type of negative regulation of protein depolymerization [GO:1901880]; negatively regulates intermediate filament depolymerization [GO:0045106] Definition: Any process that stops, prevents, or reduces the frequency, rate or extent of intermediate filament depolymerization. Note: Note that this term was split from 'negative regulation of intermediate filament polymerization and/or depolymerization ; GO:0045825' (sibling term 'negative regulation of intermediate filament polymerization ; GO:0030840').